{
  "gene_symbol": "MFSD2B",
  "term_id": "GO:0055085",
  "gene_name": "Sphingosine-1-phosphate transporter MFSD2B",
  "term_label": "transmembrane transport",
  "gene": "UniProtKB:A6NFX1"
}